G protein-coupled ATP receptor activity [GO:0045031] (molecular function) Sources: GOC:mah Relationships: is a type of G protein-coupled purinergic nucleotide receptor activity [GO:0045028] Also known as: ATP-activated nucleotide receptor activity, ATP-activated adenosine receptor activity Definition: Combining with ATP and transmitting the signal across the membrane by activating an associated G-protein; promotes the exchange of GDP for GTP on the alpha subunit of a heterotrimeric G-protein complex.